{
  "gene_name": "Carbohydrate sulfotransferase 15",
  "gene": "UniProtKB:Q7LFX5",
  "term_label": "hexose biosynthetic process",
  "gene_symbol": "CHST15",
  "term_id": "GO:0019319"
}